{
  "gene_symbol": "CFAP206",
  "gene_name": "Cilia- and flagella-associated protein 206",
  "term_label": "regulation of flagellated sperm motility",
  "term_id": "GO:1901317",
  "gene": "UniProtKB:Q8IYR0"
}